{
  "term_label": "receptor ligand activity",
  "gene_symbol": "RAET1L",
  "gene": "UniProtKB:Q5VY80",
  "term_id": "GO:0048018",
  "gene_name": "UL16-binding protein 6"
}